{
  "term_id": "GO:0005615",
  "gene_symbol": "LRG1",
  "term_label": "extracellular space",
  "gene_name": "Leucine-rich alpha-2-glycoprotein",
  "gene": "UniProtKB:P02750"
}